epithelial cell apoptotic process [GO:1904019] (biological process) References: PMID:19137015 Sources: GOC:TermGenie, GO_REF:0000085 Subtypes: type B pancreatic cell apoptotic process [GO:0097050], keratinocyte apoptotic process [GO:0097283], hepatocyte apoptotic process [GO:0097284], Sertoli cell apoptotic process [GO:1902484], cholangiocyte apoptotic process [GO:1902488], GO:1903210, GO:1904700, lens fiber cell apoptotic process [GO:1990086], epithelial cell apoptotic process involved in palatal shelf morphogenesis [GO:1990134] Definition: Any apoptotic process in an epithelial cell. Relationships: is a type of apoptotic process [GO:0006915] Regulation: regulated by regulation of epithelial cell apoptotic process [GO:1904035]; negatively regulated by negative regulation of epithelial cell apoptotic process [GO:1904036]; RO_0002213 by positive regulation of epithelial cell apoptotic process [GO:1904037] Also known as: epitheliocyte apoptotic process, epithelial cell apoptosis, epitheliocyte apoptosis